{
  "term_id": "GO:0005829",
  "gene_symbol": "PEX1",
  "gene": "UniProtKB:O43933",
  "gene_name": "Peroxisomal ATPase PEX1",
  "term_label": "cytosol"
}